{
  "gene_name": "Synaptotagmin-7",
  "term_id": "GO:0030424",
  "gene": "UniProtKB:O43581",
  "term_label": "axon",
  "gene_symbol": "SYT7"
}